{
  "gene_name": "RNA guanine-N7 methyltransferase-activating subunit-like protein",
  "gene_symbol": "RAMACL",
  "term_id": "GO:0003723",
  "gene": "UniProtKB:A0A3B3IU46",
  "term_label": "RNA binding"
}